ectodermal placode formation [GO:0060788] (biological process) Subtypes: lens placode formation [GO:0001743], GO:0001744, olfactory placode formation [GO:0030910], GO:0043049, mammary placode formation [GO:0060596], GO:0060789, GO:0060790, sebaceous gland placode formation [GO:0060791], sweat gland placode formation [GO:0060793] Relationships: is a type of anatomical structure formation involved in morphogenesis [GO:0048646]; is part of ectodermal placode morphogenesis [GO:0071697] Definition: The developmental process in which an ectodermal placode forms. An ectodermal placode is a thickening of the ectoderm that is the primordium of many structures derived from the ectoderm. Sources: GOC:dph, GOC:sdb_2009, GOC:tb